{
  "gene": "UniProtKB:P40238",
  "gene_symbol": "MPL",
  "term_label": "platelet formation",
  "gene_name": "Thrombopoietin receptor",
  "term_id": "GO:0030220"
}